{
  "term_label": "cytoplasm",
  "gene_name": "Talin-2",
  "gene": "UniProtKB:Q9Y4G6",
  "term_id": "GO:0005737",
  "gene_symbol": "TLN2"
}